{
  "gene_symbol": "MYO6",
  "gene_name": "Unconventional myosin-VI",
  "term_label": "microfilament motor activity",
  "term_id": "GO:0000146",
  "gene": "UniProtKB:Q9UM54"
}